{
  "gene_name": "Lysozyme-like protein 1",
  "gene": "UniProtKB:Q6UWQ5",
  "gene_symbol": "LYZL1",
  "term_id": "UNKNOWN:0002",
  "term_label": "Unknown biological process"
}